{
  "gene": "UniProtKB:Q8IVL0",
  "term_label": "nervous system development",
  "gene_name": "Neuron navigator 3",
  "term_id": "GO:0007399",
  "gene_symbol": "NAV3"
}